{
  "gene_symbol": "APOBEC1",
  "term_label": "cytoplasm",
  "term_id": "GO:0005737",
  "gene": "UniProtKB:P41238",
  "gene_name": "C-U-editing enzyme APOBEC-1"
}